{
  "gene": "UniProtKB:Q8N0U8",
  "gene_name": "Vitamin K epoxide reductase complex subunit 1-like protein 1",
  "term_id": "GO:0047057",
  "term_label": "vitamin-K-epoxide reductase (warfarin-sensitive) activity",
  "gene_symbol": "VKORC1L1"
}